{
  "term_id": "GO:0005737",
  "gene": "UniProtKB:Q9NY65",
  "term_label": "cytoplasm",
  "gene_symbol": "TUBA8",
  "gene_name": "Tubulin alpha-8 chain"
}